{
  "gene": "UniProtKB:Q8TEW0",
  "gene_symbol": "PARD3",
  "term_id": "GO:0008104",
  "term_label": "intracellular protein localization",
  "gene_name": "Partitioning defective 3 homolog"
}